{
  "term_id": "GO:0098632",
  "gene_name": "Netrin-G1",
  "gene": "UniProtKB:Q9Y2I2",
  "term_label": "cell-cell adhesion mediator activity",
  "gene_symbol": "NTNG1"
}